{
  "term_label": "phosphatidylinositol binding",
  "gene_symbol": "ITPR2",
  "gene": "UniProtKB:Q14571",
  "gene_name": "Inositol 1,4,5-trisphosphate receptor type 2",
  "term_id": "GO:0035091"
}